cellobiose phosphorylase activity [GO:0047738] (molecular function) Relationships: is_a 1,4-alpha-oligoglucan phosphorylase activity [GO:0004645] Sources: RHEA:19493 Definition: Catalysis of the reaction: cellobiose + phosphate = alpha-D-glucose 1-phosphate + D-glucose. Also known as: cellobiose:phosphate alpha-D-glucosyltransferase activity